{
  "term_id": "UNKNOWN:0003",
  "gene": "UniProtKB:Q9ULL5",
  "term_label": "Unknown cellular component",
  "gene_name": "Proline-rich protein 12",
  "gene_symbol": "PRR12"
}